{
  "gene_symbol": "CDK11B",
  "gene_name": "Cyclin-dependent kinase 11B",
  "gene": "UniProtKB:P21127",
  "term_label": "protein serine/threonine kinase activity",
  "term_id": "GO:0004674"
}